{
  "term_label": "nucleus",
  "gene_name": "Zinc finger protein 792",
  "gene": "UniProtKB:Q3KQV3",
  "gene_symbol": "ZNF792",
  "term_id": "GO:0005634"
}